{
  "term_label": "Unknown molecular function",
  "gene": "UniProtKB:Q96EZ4",
  "term_id": "UNKNOWN:0001",
  "gene_symbol": "MYEOV",
  "gene_name": "Myeloma-overexpressed gene protein"
}